{
  "gene_symbol": "OPRD1",
  "term_id": "GO:0038046",
  "gene_name": "Delta-type opioid receptor",
  "gene": "UniProtKB:P41143",
  "term_label": "G protein-coupled enkephalin receptor activity"
}